thiosulfate-thioredoxin sulfurtransferase activity [GO:0103041] (molecular function) Sources: GOC:pz, RHEA:83859 Definition: Catalysis of the reaction: thiosulfate + [thioredoxin]-dithiol = sulfite + 2 H+ + [thioredoxin]-disulfide + hydrogen sulfide. Relationships: is a type of sulfurtransferase activity [GO:0016783]